{
  "gene": "UniProtKB:Q8N3J6",
  "gene_name": "Cell adhesion molecule 2",
  "term_label": "neuronal cell body membrane",
  "gene_symbol": "CADM2",
  "term_id": "GO:0032809"
}